{
  "gene": "UniProtKB:Q6UXN8",
  "term_label": "receptor-mediated endocytosis",
  "gene_symbol": "CLEC9A",
  "term_id": "GO:0006898",
  "gene_name": "C-type lectin domain family 9 member A"
}